{
  "gene_name": "Dolichol-phosphate mannosyltransferase subunit 1",
  "term_id": "GO:0005789",
  "gene_symbol": "DPM1",
  "term_label": "endoplasmic reticulum membrane",
  "gene": "UniProtKB:O60762"
}